{
  "gene": "UniProtKB:Q9UKK6",
  "gene_symbol": "NXT1",
  "term_id": "UNKNOWN:0001",
  "term_label": "Unknown molecular function",
  "gene_name": "NTF2-related export protein 1"
}